{
  "gene_name": "Triosephosphate isomerase",
  "term_id": "GO:0005829",
  "gene": "UniProtKB:P60174",
  "term_label": "cytosol",
  "gene_symbol": "TPI1"
}